nicotinamidase activity [GO:0008936] (molecular function) Definition: Catalysis of the reaction: nicotinamide + H2O = nicotinate + NH4+. Sources: RHEA:14545 Relationships: is a type of amidase activity [GO:0004040] Also known as: NAMase activity, YNDase activity, nicotinamide amidase activity, nicotinamide amidohydrolase activity, nicotinamide deaminase activity, nicotine deamidase activity